{
  "gene_name": "Ephrin type-B receptor 4",
  "gene": "UniProtKB:P54760",
  "term_label": "angiogenesis",
  "gene_symbol": "EPHB4",
  "term_id": "GO:0001525"
}